mannose to fructose-6-phosphate catabolic process [GO:0061611] (biological process) Relationships: is a type of fructose 6-phosphate metabolic process [GO:0006002]; is a type of GO:0019309; has part GO:0004476; BFO_0000051 mannokinase activity [GO:0019158] Sources: GOC:dph, ISBN:0201090910, ISBN:0879010479 Also known as: mannose metabolism to fructose-6-phosphate Definition: The chemical reactions and pathways in which mannose, the aldohexose manno-hexose, is converted to fructose-6-phosphate.